{
  "term_id": "UNKNOWN:0002",
  "gene": "UniProtKB:Q00LT1",
  "gene_symbol": "PRCD",
  "term_label": "Unknown biological process",
  "gene_name": "Photoreceptor disk component PRCD"
}